{
  "gene_symbol": "PAGE3",
  "gene": "UniProtKB:Q5JUK9",
  "term_id": "UNKNOWN:0003",
  "gene_name": "P antigen family member 3",
  "term_label": "Unknown cellular component"
}